capsule poly-gamma-glutamate biosynthetic process [GO:0070502] (biological process) Also known as: capsular poly-gamma-glutamate biosynthetic process, capsule poly-gamma-glutamate anabolism, capsule poly-gamma-glutamate biosynthesis, capsule poly-gamma-glutamate formation, capsule poly-gamma-glutamate synthesis References: PMID:16689787 Sources: GOC:mah Definition: The chemical reactions and pathways resulting in the formation of poly-gamma-glutamate, a polymer of D- and/or L-glutamic acid residues linked by gamma-peptidyl bonds, that forms all or part of a bacterial capsule. Relationships: is a type of capsule organization [GO:0045230]; is a type of GO:0070501